dermatan sulfate proteoglycan metabolic process [GO:0050655] (biological process) Definition: The chemical reactions and pathways involving dermatan sulfate proteoglycans, which consist of a core protein linked to a dermatan sulfate glycosaminoglycan. The dermatan sulfate chain is composed of the repeating disaccharide unit beta-(1,4)-D-hexuronic acid-beta-(1,3)-N-acetyl-D-galactosamine. The former can be a mixture of sulfated and nonsulfated D-glucuronic and L-iduronic acids, and the latter can be O-sulfated. References: PMID:17239763 Also known as: chondroitin sulfate B proteoglycan metabolic process, chondroitin sulfate B proteoglycan metabolism, dermatan sulfate proteoglycan metabolism, dermatan sulphate proteoglycan metabolic process, dermatan sulphate proteoglycan metabolism Relationships: is a type of proteoglycan metabolic process [GO:0006029] Subtypes: dermatan sulfate proteoglycan catabolic process [GO:0030209], dermatan sulfate proteoglycan biosynthetic process [GO:0050651]